{
  "gene": "UniProtKB:P31274",
  "term_id": "GO:0048704",
  "gene_symbol": "HOXC9",
  "term_label": "embryonic skeletal system morphogenesis",
  "gene_name": "Homeobox protein Hox-C9"
}